{
  "term_id": "GO:0005096",
  "term_label": "GTPase activator activity",
  "gene": "UniProtKB:Q8N264",
  "gene_name": "Rho GTPase-activating protein 24",
  "gene_symbol": "ARHGAP24"
}